{
  "gene_name": "Proton-coupled amino acid transporter 1",
  "gene": "UniProtKB:Q7Z2H8",
  "term_id": "GO:0015808",
  "gene_symbol": "SLC36A1",
  "term_label": "L-alanine transport"
}